{
  "term_label": "nervous system development",
  "term_id": "GO:0007399",
  "gene_symbol": "RXRB",
  "gene_name": "Retinoic acid receptor RXR-beta",
  "gene": "UniProtKB:P28702"
}